{
  "term_label": "platelet formation",
  "gene_name": "C-type lectin domain family 1 member B",
  "gene": "UniProtKB:Q9P126",
  "term_id": "GO:0030220",
  "gene_symbol": "CLEC1B"
}